{
  "term_label": "angiotensin maturation",
  "gene_symbol": "ANPEP",
  "gene": "UniProtKB:P15144",
  "term_id": "GO:0002003",
  "gene_name": "Aminopeptidase N"
}